{
  "gene": "UniProtKB:Q8N9R6",
  "gene_symbol": "CDRT4",
  "term_id": "UNKNOWN:0001",
  "term_label": "Unknown molecular function",
  "gene_name": "CMT1A duplicated region transcript 4 protein"
}